{
  "gene": "UniProtKB:P51946",
  "term_id": "GO:0070985",
  "gene_name": "Cyclin-H",
  "gene_symbol": "CCNH",
  "term_label": "transcription factor TFIIK complex"
}